positive regulation of cell-substrate junction organization [GO:0150117] (biological process) Sources: GOC:aruk Subtypes: positive regulation of focal adhesion assembly [GO:0051894], GO:0120183 Definition: Any process that activates or increases the frequency, rate or extent of cell-substrate junction organization. Relationships: is a type of GO:0051130; is a type of GO:0150116; positively regulates cell-substrate junction organization [GO:0150115]